regulation of neutrophil mediated killing of bacterium [GO:0070950] (biological process) Relationships: is a type of regulation of neutrophil mediated killing of symbiont cell [GO:0070949]; regulates neutrophil-mediated killing of bacterium [GO:0070944] Subtypes: regulation of neutrophil mediated killing of gram-negative bacterium [GO:0070951], regulation of neutrophil mediated killing of gram-positive bacterium [GO:0070952], negative regulation of neutrophil mediated killing of bacterium [GO:0070956], positive regulation of neutrophil mediated killing of bacterium [GO:0070962] Definition: Any process that modulates the rate, frequency or extent of neutrophil mediated killing of a bacterium, the directed killing of a bacterium by a neutrophil. Sources: GOC:add, GOC:mah